{
  "gene_symbol": "FOXD4L5",
  "gene": "UniProtKB:Q5VV16",
  "term_label": "RNA polymerase II cis-regulatory region sequence-specific DNA binding",
  "gene_name": "Forkhead box protein D4-like 5",
  "term_id": "GO:0000978"
}